{
  "gene_symbol": "INHBA",
  "term_label": "extracellular space",
  "term_id": "GO:0005615",
  "gene": "UniProtKB:P08476",
  "gene_name": "Inhibin beta A chain"
}